tube development [GO:0035295] (BP) Definition: The process whose specific outcome is the progression of a tube over time, from its initial formation to a mature structure. Epithelial and endothelial tubes transport gases, liquids and cells from one site to another and form the basic structure of many organs and tissues including lung and trachea, kidney, the mammary gland, the vascular system and the gastrointestinal and urinary-genital tracts. References: PMID:12526790 Relationships: is a type of anatomical structure development [GO:0048856]; is part of multicellular organism development [GO:0007275] Subtypes: neural tube development [GO:0021915], GO:0030323, embryonic heart tube development [GO:0035050], GO:0035502, ureter part of ureteric bud development [GO:0035503], digestive tract development [GO:0048565], oviduct development [GO:0060066], GO:0060872, common bile duct development [GO:0061009], urethra epithelium development [GO:0061071], seminal vesicle epithelium development [GO:0061108], paramesonephric duct development [GO:0061205], renal tubule development [GO:0061326], otic vesicle development [GO:0071599], GO:0072031, proximal convoluted tubule segment 2 development [GO:0072032], collecting duct development [GO:0072044], long descending thin limb bend development [GO:0072065], prebend segment development [GO:0072066], mesonephric tubule development [GO:0072164], metanephric tubule development [GO:0072170], nephric duct development [GO:0072176], ureter development [GO:0072189], seminiferous tubule development [GO:0072520], GO:1905867